2-hydroxybenzoyl-CoA catabolic process [GO:1901886] (biological process) References: PMID:19757094 Sources: GOC:TermGenie Relationships: is a type of GO:0006637; is a type of GO:0019336; is a type of sulfur compound catabolic process [GO:0044273]; is a type of purine-containing compound catabolic process [GO:0072523]; is_a nucleoside phosphate catabolic process [GO:1901292] Also known as: 2-hydroxybenzoyl-CoA breakdown, 2-hydroxybenzoyl-CoA catabolism, 2-hydroxybenzoyl-CoA degradation Definition: The chemical reactions and pathways resulting in the breakdown of 2-hydroxybenzoyl-CoA.